{
  "gene": "UniProtKB:A6NGG3",
  "term_id": "UNKNOWN:0002",
  "term_label": "Unknown biological process",
  "gene_symbol": "LINC03041",
  "gene_name": "Putative uncharacterized protein encoded by LINC03041"
}